{
  "term_id": "GO:0019901",
  "gene": "UniProtKB:O94844",
  "term_label": "protein kinase binding",
  "gene_name": "Rho-related BTB domain-containing protein 1",
  "gene_symbol": "RHOBTB1"
}